corticospinal neuron axon guidance through the internal capsule [GO:0021968] (biological process) Also known as: corticospinal neuron axon pathfinding through the internal capsule Relationships: is a type of axon guidance [GO:0007411]; is part of corticospinal neuron axon guidance [GO:0021966] Definition: The process in which the migration of an axon growth cone of a pyramidal cell that is part of the corticospinal tract is directed after exiting the cerebral cortex through the internal capsule in response to a combination of attractive and repulsive cues. References: PMID:9878731 Sources: GOC:cls, GOC:dgh, GOC:dph, GOC:jid, GO_REF:0000021